{
  "gene": "UniProtKB:Q9UMR7",
  "gene_symbol": "CLEC4A",
  "gene_name": "C-type lectin domain family 4 member A",
  "term_id": "GO:0038187",
  "term_label": "pattern recognition receptor activity"
}